{
  "term_label": "Unknown cellular component",
  "gene_symbol": "SPANXD",
  "gene_name": "Sperm protein associated with the nucleus on the X chromosome D",
  "term_id": "UNKNOWN:0003",
  "gene": "UniProtKB:Q9BXN6"
}